{
  "gene_symbol": "APOBEC3H",
  "term_id": "GO:0000932",
  "gene_name": "DNA dC-dU-editing enzyme APOBEC-3H",
  "gene": "UniProtKB:Q6NTF7",
  "term_label": "P-body"
}